{
  "gene": "UniProtKB:Q6URK8",
  "term_id": "UNKNOWN:0001",
  "gene_symbol": "SPMIP8",
  "gene_name": "Testis, prostate and placenta-expressed protein",
  "term_label": "Unknown molecular function"
}